{
  "gene_symbol": "TLR7",
  "gene": "UniProtKB:Q9NYK1",
  "gene_name": "Toll-like receptor 7",
  "term_id": "GO:0038187",
  "term_label": "pattern recognition receptor activity"
}